{
  "term_label": "Unknown biological process",
  "gene": "UniProtKB:Q8IV38",
  "term_id": "UNKNOWN:0002",
  "gene_name": "Ankyrin repeat and MYND domain-containing protein 2",
  "gene_symbol": "ANKMY2"
}